delta1-piperideine-2-carboxylate reductase activity [GO:0047125] (molecular function) Relationships: is a type of GO:0016646 Also known as: D1-piperideine-2-carboxylate reductase activity, delta 1-piperideine-2-carboxylate reductase activity, 1,2-didehydropipecolate reductase activity, 1,2-didehydropipecolic reductase activity, L-pipecolate:NADP+ 2-oxidoreductase activity, P2C reductase activity Sources: EC:1.5.1.21 Definition: Catalysis of the reaction: NADP+ + L-pipecolate = NADPH + delta1-piperideine-2-carboxylate.